{
  "term_label": "DNA-binding transcription factor activity, RNA polymerase II-specific",
  "gene_name": "Forkhead box protein D3",
  "term_id": "GO:0000981",
  "gene": "UniProtKB:Q9UJU5",
  "gene_symbol": "FOXD3"
}